{
  "gene_symbol": "IQCK",
  "term_label": "Unknown biological process",
  "gene": "UniProtKB:Q8N0W5",
  "gene_name": "IQ domain-containing protein K",
  "term_id": "UNKNOWN:0002"
}